{
  "gene_symbol": "RIT2",
  "term_label": "plasma membrane",
  "gene": "UniProtKB:Q99578",
  "term_id": "GO:0005886",
  "gene_name": "GTP-binding protein Rit2"
}